gene conversion at mating-type locus [GO:0007534] (biological process) References: PMID:10716938, PMID:7646483, PMID:9928492 Sources: GOC:elh Also known as: strand invasion involved in gene conversion at mating-type locus, gene conversion at mating-type locus, DNA double-strand break formation, gene conversion at mating-type locus, DNA double-strand break processing, gene conversion at mating-type locus, DNA repair synthesis, gene conversion at mating-type locus, termination of copy-synthesis, heteroduplex formation involved in gene conversion at mating-type locus Relationships: is a type of mitotic recombination [GO:0006312]; is a type of gene conversion [GO:0035822]; is part of mating type switching [GO:0007533]; has part DNA double-strand break processing [GO:0000729]; has part DNA synthesis involved in DNA repair [GO:0000731]; has part heteroduplex formation [GO:0030491]; has part GO:0042148; has part site-specific DNA replication termination [GO:0071170] Definition: The conversion of the mating-type locus from one allele to another resulting from the recombinational repair of a site-specific double-strand break at the mating-type locus with information from a silent donor sequence. There is no reciprocal exchange of information because the mating-type locus copies information from the donor sequence and the donor sequence remains unchanged.